{
  "gene": "UniProtKB:Q9BYZ8",
  "term_label": "extracellular space",
  "term_id": "GO:0005615",
  "gene_name": "Regenerating islet-derived protein 4",
  "gene_symbol": "REG4"
}